{
  "term_label": "RNA polymerase I complex",
  "term_id": "GO:0005736",
  "gene_symbol": "POLR1H",
  "gene": "UniProtKB:Q9P1U0",
  "gene_name": "DNA-directed RNA polymerase I subunit RPA12"
}